{
  "gene_symbol": "PIK3CG",
  "term_id": "GO:0043491",
  "term_label": "phosphatidylinositol 3-kinase/protein kinase B signal transduction",
  "gene": "UniProtKB:P48736",
  "gene_name": "Phosphatidylinositol 4,5-bisphosphate 3-kinase catalytic subunit gamma isoform"
}